dichotomous subdivision of terminal units involved in lung branching [GO:0060448] (biological process) Sources: GOC:dph, GOC:mtg_lung Subtypes: orthogonal dichotomous subdivision of terminal units involved in lung branching morphogenesis [GO:0060488], planar dichotomous subdivision of terminal units involved in lung branching morphogenesis [GO:0060489] Definition: The process in which a lung bud bifurcates. Relationships: is a type of GO:0060600; is part of epithelial tube branching involved in lung morphogenesis [GO:0060441] Also known as: bud bifurcation involved in lung branching